acetylglutamate kinase activity [GO:0003991] (molecular function) Sources: EC:2.7.2.8 Definition: Catalysis of the reaction: ATP + N-acetyl-L-glutamate = ADP + N-acetyl-L-glutamate-5-phosphate. Also known as: ATP:N-acetyl-L-glutamate 5-phosphotransferase activity, N-acetylglutamate 5-phosphotransferase activity, N-acetylglutamate kinase activity, N-acetylglutamate phosphokinase activity, N-acetylglutamic 5-phosphotransferase activity, acetylglutamate phosphokinase activity Regulation: regulated by acetylglutamate kinase regulator activity [GO:0010307] Relationships: is_a kinase activity [GO:0016301]; is_a GO:0016774